{
  "gene_name": "Calcium and integrin-binding family member 2",
  "gene": "UniProtKB:O75838",
  "term_label": "cytoplasm",
  "term_id": "GO:0005737",
  "gene_symbol": "CIB2"
}